{
  "term_id": "GO:0004714",
  "gene_symbol": "EGFR",
  "gene_name": "Epidermal growth factor receptor",
  "gene": "UniProtKB:P00533",
  "term_label": "transmembrane receptor protein tyrosine kinase activity"
}